{
  "term_id": "GO:0005930",
  "gene": "UniProtKB:Q8NDM7",
  "gene_name": "Cilia- and flagella-associated protein 43",
  "gene_symbol": "CFAP43",
  "term_label": "axoneme"
}